L-lactate dehydrogenase (cytochrome) activity [GO:0004460] (molecular function) Also known as: L-lactate dehydrogenase activity, lactic acid dehydrogenase activity, (S)-lactate:ferricytochrome-c 2-oxidoreductase activity, L(+)-lactate:cytochrome c oxidoreductase activity, L-lactate cytochrome c oxidoreductase activity, L-lactate cytochrome c reductase activity, L-lactate ferricytochrome c oxidoreductase activity, cytochrome b2, cytochrome b2 (flavin-free derivative of flavocytochrome b2), dehydrogenase, lactate (cytochrome), flavocytochrome b2, lactate dehydrogenase (cytochrome), lactic cytochrome c reductase activity Definition: Catalysis of the reaction: (S)-lactate + 2 [Fe(III)cytochrome c] = 2 [Fe(II)cytochrome c] + 2 H+ + pyruvate. Sources: RHEA:19909 Relationships: is a type of oxidoreductase activity, acting on the CH-OH group of donors, cytochrome as acceptor [GO:0016898]; is a type of GO:0140171